{
  "term_label": "proteolysis involved in protein catabolic process",
  "gene": "UniProtKB:O60911",
  "gene_symbol": "CTSV",
  "term_id": "GO:0051603",
  "gene_name": "Cathepsin L2"
}